{
  "term_label": "proteolysis",
  "term_id": "GO:0006508",
  "gene_symbol": "CTSE",
  "gene_name": "Cathepsin E",
  "gene": "UniProtKB:P14091"
}